neuronal ion channel clustering [GO:0045161] (biological process) Subtypes: clustering of voltage-gated sodium channels [GO:0045162], clustering of voltage-gated potassium channels [GO:0045163], clustering of voltage-gated calcium channels [GO:0070073] Relationships: is a type of GO:0061024; is part of neuron maturation [GO:0042551] References: PMID:11456440 Definition: The process in which voltage-gated ion channels become localized to distinct subcellular domains in the neuron. Specific targeting, clustering, and maintenance of these channels in their respective domains are essential to achieve high conduction velocities of action potential propagation.